{
  "gene": "UniProtKB:Q5VVC0",
  "term_id": "GO:0007131",
  "gene_symbol": "SPO16",
  "term_label": "reciprocal meiotic recombination",
  "gene_name": "Protein SPO16 homolog"
}